{
  "term_label": "bicarbonate transmembrane transporter activity",
  "gene_name": "Putative solute carrier family 26 member 10P",
  "gene": "UniProtKB:Q8NG04",
  "term_id": "GO:0015106",
  "gene_symbol": "SLC26A10P"
}